{
  "gene_symbol": "SCRIB",
  "gene": "UniProtKB:Q14160",
  "term_label": "neurotransmitter receptor transport, endosome to postsynaptic membrane",
  "gene_name": "Protein scribble homolog",
  "term_id": "GO:0098887"
}